{
  "term_id": "GO:0050911",
  "gene_name": "Olfactory receptor 10G3",
  "gene_symbol": "OR10G3",
  "gene": "UniProtKB:Q8NGC4",
  "term_label": "detection of chemical stimulus involved in sensory perception of smell"
}